angiotensin-mediated vasodilation involved in regulation of systemic arterial blood pressure [GO:0002033] (BP) Definition: The process that increases the diameter of a blood vessel via the renin-angiotensin system. Relationships: is a type of negative regulation of systemic arterial blood pressure [GO:0003085]; is a type of vasodilation [GO:0042311]; BFO_0000050 maintenance of blood vessel diameter homeostasis by renin-angiotensin [GO:0002034] Also known as: vasodilation by angiotensin involved in regulation of systemic arterial blood pressure References: PMID:10425188 Sources: GOC:pr, ISBN:0323031951